{
  "term_label": "negative regulation of autophagosome maturation",
  "gene_name": "PHD finger protein 23",
  "gene_symbol": "PHF23",
  "gene": "UniProtKB:Q9BUL5",
  "term_id": "GO:1901097"
}